{
  "term_id": "GO:0017154",
  "gene_name": "Plexin-A1",
  "gene_symbol": "PLXNA1",
  "term_label": "semaphorin receptor activity",
  "gene": "UniProtKB:Q9UIW2"
}